{
  "term_id": "UNKNOWN:0001",
  "gene": "UniProtKB:Q3ZAQ7",
  "term_label": "Unknown molecular function",
  "gene_symbol": "VMA21",
  "gene_name": "Vacuolar ATPase assembly integral membrane protein VMA21"
}